{
  "gene_name": "Toll-like receptor 4",
  "term_id": "GO:0034142",
  "gene": "UniProtKB:O00206",
  "term_label": "toll-like receptor 4 signaling pathway",
  "gene_symbol": "TLR4"
}